{
  "gene_symbol": "PIPOX",
  "term_id": "GO:0033514",
  "gene_name": "Peroxisomal sarcosine oxidase",
  "term_label": "L-lysine catabolic process to acetyl-CoA via L-pipecolate",
  "gene": "UniProtKB:Q9P0Z9"
}